{
  "term_label": "Unknown cellular component",
  "gene_name": "Neurofibromin",
  "gene": "UniProtKB:P21359",
  "term_id": "UNKNOWN:0003",
  "gene_symbol": "NF1"
}